{
  "gene_name": "Macoilin",
  "term_label": "chemotaxis",
  "gene_symbol": "MACO1",
  "term_id": "GO:0006935",
  "gene": "UniProtKB:Q8N5G2"
}